negative regulation of organelle assembly [GO:1902116] (biological process) Subtypes: negative regulation of cytoplasmic mRNA processing body assembly [GO:0010607], GO:0046600, GO:0060299, negative regulation of stress granule assembly [GO:0062030], negative regulation of pseudohyphal septin ring assembly [GO:0062166], negative regulation of podosome assembly [GO:0071802], negative regulation of postsynaptic density assembly [GO:0160037], GO:1900504, negative regulation of cilium assembly [GO:1902018], negative regulation of bacterial-type flagellum assembly [GO:1902209], negative regulation of autophagosome assembly [GO:1902902], negative regulation of extracellular exosome assembly [GO:1903552], negative regulation of gut granule assembly [GO:1904756], negative regulation of cardiac myofibril assembly [GO:1905305], negative regulation of kinetochore assembly [GO:1905560], negative regulation of spindle assembly [GO:1905831] Relationships: is a type of negative regulation of organelle organization [GO:0010639]; is a type of regulation of organelle assembly [GO:1902115]; negatively regulates organelle assembly [GO:0070925] Also known as: down regulation of organelle assembly, down-regulation of organelle assembly, downregulation of organelle assembly, inhibition of organelle assembly Sources: GOC:TermGenie, GOC:pr Definition: Any process that stops, prevents or reduces the frequency, rate or extent of organelle assembly.